{
  "gene_symbol": "KIR2DS2",
  "gene_name": "Killer cell immunoglobulin-like receptor 2DS2",
  "term_id": "GO:0002767",
  "term_label": "immune response-inhibiting cell surface receptor signaling pathway",
  "gene": "UniProtKB:P43631"
}